{
  "gene_name": "Amyloid beta precursor protein binding family B member 2",
  "gene": "UniProtKB:Q92870",
  "term_id": "GO:0006355",
  "gene_symbol": "APBB2",
  "term_label": "regulation of DNA-templated transcription"
}